{
  "term_label": "myosin phosphatase regulator activity",
  "gene_symbol": "PPP1R16B",
  "gene": "UniProtKB:Q96T49",
  "term_id": "GO:0017020",
  "gene_name": "Protein phosphatase 1 regulatory inhibitor subunit 16B"
}